{
  "gene_name": "Epithelial discoidin domain-containing receptor 1",
  "term_id": "GO:0043235",
  "term_label": "receptor complex",
  "gene_symbol": "DDR1",
  "gene": "UniProtKB:Q08345"
}